G protein activity [GO:0003925] (molecular function) References: PMID:16923326, PMID:24470015 Definition: A molecular function regulator that cycles between active GTP-bound and inactive GDP-bound states. In its active state, binds to a variety of effector proteins to regulate cellular processes. Intrinsic GTPase activity returns the G protein to its GDP-bound state. The return to the GDP-bound state can be accelerated by the action of a GTPase-activating protein (GAP). Relationships: is a type of GTPase activity [GO:0003924]; is a type of GO:0098772 Also known as: signaling G protein activity, Ras superfamily protein, heterotrimeric G-protein GTPase activity, large G-protein GTPase activity, large G-protein activity, small G-protein, small GTPase, small GTPase activity, small monomeric G protein activity, small monomeric GTPase activity